sodium-dependent organic anion transport [GO:0043251] (biological process) Sources: GOC:go_curators Relationships: is a type of organic anion transport [GO:0015711] Definition: The directed, sodium-dependent, movement of organic anions into, out of or within a cell, or between cells, by means of some agent such as a transporter or pore.